phosphatidylinositol 3-kinase activator activity [GO:0141038] (molecular function) References: PMID:31686003 Definition: Binds to and increases the activity of a phosphatidylinositol 3-kinase (PI3K). Relationships: is a type of phosphatidylinositol 3-kinase regulator activity [GO:0035014]